{
  "term_id": "GO:0070527",
  "gene_symbol": "FGG",
  "term_label": "platelet aggregation",
  "gene": "UniProtKB:P02679",
  "gene_name": "Fibrinogen gamma chain"
}